poly(hydroxyalkanoate) biosynthetic process from glucose [GO:1902924] (biological process) References: PMID:24425304 Sources: GOC:TermGenie, GOC:mengo_curators, GO_REF:0000092 Also known as: poly(hydroxyalkanoate) anabolism from glucose, poly(hydroxyalkanoate) biosynthesis from glucose, poly(hydroxyalkanoate) formation from glucose, poly(hydroxyalkanoate) synthesis from glucose Definition: The chemical reactions and pathways resulting in the formation of poly(hydroxyalkanoate) from glucose. Relationships: is a type of GO:0006006; is a type of GO:1901441